regulation of synaptic plasticity by receptor localization to synapse [GO:1900383] (biological process) Definition: Any process that modulates synaptic plasticity, the ability of synapses to change as circumstances require, via receptor localization to the synapse, the junction between a nerve fiber of one neuron and another neuron or muscle fiber or glial cell. Processes may include receptor transport to, and/or maintenance at, the synapse. Relationships: is a type of GO:0097120 Also known as: regulation of synaptic plasticity by receptor localisation to synapse References: PMID:22464329 Sources: GOC:TermGenie, GOC:kmv